{
  "term_label": "DNA recombination",
  "gene_symbol": "TOP3B",
  "gene": "UniProtKB:O95985",
  "term_id": "GO:0006310",
  "gene_name": "DNA topoisomerase 3-beta-1"
}